regulation of cellular response to glucose starvation [GO:1904547] (biological process) Definition: Any process that modulates the frequency, rate or extent of cellular response to glucose starvation. References: PMID:21118717 Sources: GOC:TermGenie, GO_REF:0000058 Relationships: is a type of regulation of response to nutrient levels [GO:0032107]; is a type of GO:0080135; regulates cellular response to glucose starvation [GO:0042149]